{
  "gene_symbol": "CASZ1",
  "term_id": "GO:0045664",
  "term_label": "regulation of neuron differentiation",
  "gene_name": "Zinc finger protein castor homolog 1",
  "gene": "UniProtKB:Q86V15"
}